{
  "gene": "UniProtKB:Q9UI26",
  "gene_symbol": "IPO11",
  "term_id": "GO:0061608",
  "gene_name": "Importin-11",
  "term_label": "nuclear import signal receptor activity"
}